{
  "term_id": "GO:0005737",
  "term_label": "cytoplasm",
  "gene_name": "Parkinson disease protein 7",
  "gene": "UniProtKB:Q99497",
  "gene_symbol": "PARK7"
}